eye photoreceptor cell development [GO:0042462] (biological process) Sources: GOC:jl, ISBN:0192800981 Regulation: regulated by regulation of eye photoreceptor cell development [GO:0042478]; positively regulated by GO:0042479; negatively regulated by negative regulation of eye photoreceptor cell development [GO:0042480] Definition: Development of a photoreceptor, a sensory cell in the eye that reacts to the presence of light. They usually contain a pigment that undergoes a chemical change when light is absorbed, thus stimulating a nerve. Subtypes: compound eye photoreceptor development [GO:0042051], GO:0046548, retinal cone cell development [GO:0046549], camera-type eye photoreceptor cell development [GO:0062139] Relationships: is a type of photoreceptor cell development [GO:0042461]; is part of eye photoreceptor cell differentiation [GO:0001754]